{
  "term_id": "GO:0015840",
  "term_label": "urea transport",
  "gene": "UniProtKB:O75631",
  "gene_name": "Uroplakin-3a",
  "gene_symbol": "UPK3A"
}